pseudohyphal septin ring assembly [GO:0062163] (biological process) References: PMID:29567712 Regulation: regulated by regulation of pseudohyphal septin ring assembly [GO:0062164]; positively regulated by GO:0062165; negatively regulated by GO:0062166 Definition: The aggregation, arrangement and bonding together of septins and associated proteins to form a tight ring-shaped structure that forms in the division plane at the junction between the mother cell and a pseudohyphal projection. Relationships: is a type of GO:0000921